{
  "gene_symbol": "ZNF28",
  "gene": "UniProtKB:P17035",
  "term_id": "GO:0006357",
  "term_label": "regulation of transcription by RNA polymerase II",
  "gene_name": "Zinc finger protein 28"
}